{
  "gene_name": "Neurexin-2",
  "term_id": "GO:0005886",
  "gene": "UniProtKB:Q9P2S2",
  "gene_symbol": "NRXN2",
  "term_label": "plasma membrane"
}